regulation of connective tissue replacement involved in inflammatory response wound healing [GO:1904596] (biological process) Definition: Any process that modulates the frequency, rate or extent of wound healing connective tissue replacement, which may be replaced with fibrotic material, that occurs as part of an inflammatory response. Relationships: is a type of regulation of connective tissue replacement [GO:1905203]; regulates connective tissue replacement involved in inflammatory response wound healing [GO:0002248] Subtypes: negative regulation of connective tissue replacement involved in inflammatory response wound healing [GO:1904597], GO:1904598 References: PMID:18245812 Sources: GOC:TermGenie, GOC:krc, GO_REF:0000058 Also known as: regulation of fibrosis during inflammatory response, regulation of connective tissue replacement during inflammatory response